{
  "term_label": "DNA-binding transcription factor activity, RNA polymerase II-specific",
  "gene": "UniProtKB:P15863",
  "gene_name": "Paired box protein Pax-1",
  "gene_symbol": "PAX1",
  "term_id": "GO:0000981"
}